{
  "term_label": "Unknown molecular function",
  "gene_symbol": "HUS1",
  "gene": "UniProtKB:O60921",
  "term_id": "UNKNOWN:0001",
  "gene_name": "Checkpoint protein HUS1"
}